{
  "gene_name": "Leukocyte receptor cluster member 1",
  "gene_symbol": "LENG1",
  "term_id": "UNKNOWN:0001",
  "gene": "UniProtKB:Q96BZ8",
  "term_label": "Unknown molecular function"
}